{
  "gene_symbol": "GAL3ST1",
  "term_label": "Unknown cellular component",
  "gene": "UniProtKB:Q99999",
  "gene_name": "Galactosylceramide sulfotransferase",
  "term_id": "UNKNOWN:0003"
}